{
  "gene_name": "Regulator of G-protein signaling 4",
  "gene": "UniProtKB:P49798",
  "term_id": "GO:0045744",
  "term_label": "negative regulation of G protein-coupled receptor signaling pathway",
  "gene_symbol": "RGS4"
}